DNA strand exchange activator activity [GO:0140619] (MF) Definition: Binds to and increases a DNA strand exchange activity. References: PMID:33493431 Relationships: is a type of enzyme activator activity [GO:0008047]; positively regulates GO:0000150